{
  "gene_name": "Lymphocyte antigen 96",
  "term_label": "positive regulation of lipopolysaccharide-mediated signaling pathway",
  "term_id": "GO:0031666",
  "gene": "UniProtKB:Q9Y6Y9",
  "gene_symbol": "LY96"
}